tetracycline biosynthetic process [GO:0043644] (biological process) Definition: The chemical reactions and pathways resulting in the formation of tetracycline, (4S,4aS,5aS,6S,12aS)-4-(dimethylamino)-3,6,10,12,12a-pentahydroxy-6-methyl-1,11-dioxo-1,4,4a,5,5a,6,11,12a-octahydrotetracene-2-carboxamide, a broad-spectrum antibiotic produced by streptomyces bacteria that blocks binding of aminoacyl tRNA to the ribosomes of both Gram-positive and Gram-negative organisms (and those of organelles). Sources: GOC:jl, Wikipedia:Tetracycline Relationships: is a type of antibiotic biosynthetic process [GO:0017000]; is a type of GO:0030639; is a type of ketone biosynthetic process [GO:0042181]; is a type of tertiary alcohol biosynthetic process [GO:1902645] Also known as: tetracyclin biosynthesis, tetracyclin biosynthetic process